{
  "term_label": "positive regulation of transcription by RNA polymerase II",
  "gene_symbol": "KMT2C",
  "term_id": "GO:0045944",
  "gene": "UniProtKB:Q8NEZ4",
  "gene_name": "Histone-lysine N-methyltransferase 2C"
}